{
  "gene_symbol": "SLC41A1",
  "term_label": "plasma membrane",
  "gene": "UniProtKB:Q8IVJ1",
  "gene_name": "Solute carrier family 41 member 1",
  "term_id": "GO:0005886"
}